{
  "term_id": "GO:0000981",
  "gene_symbol": "ZSCAN5DP",
  "gene_name": "Putative zinc finger and SCAN domain-containing protein 5D",
  "term_label": "DNA-binding transcription factor activity, RNA polymerase II-specific",
  "gene": "UniProtKB:P0CG00"
}